{
  "gene": "UniProtKB:O95817",
  "gene_name": "BAG family molecular chaperone regulator 3",
  "gene_symbol": "BAG3",
  "term_id": "GO:0005829",
  "term_label": "cytosol"
}